{
  "term_id": "UNKNOWN:0001",
  "gene_name": "Keratin-associated protein 10-6",
  "term_label": "Unknown molecular function",
  "gene": "UniProtKB:P60371",
  "gene_symbol": "KRTAP10-6"
}